{
  "gene": "UniProtKB:Q9NY57",
  "gene_symbol": "STK32B",
  "gene_name": "Serine_threonine-protein kinase 32B",
  "term_label": "protein serine/threonine kinase activity",
  "term_id": "GO:0004674"
}